{
  "gene": "UniProtKB:P00709",
  "gene_name": "Alpha-lactalbumin",
  "term_label": "defense response to Gram-negative bacterium",
  "gene_symbol": "LALBA",
  "term_id": "GO:0050829"
}